{
  "term_label": "negative regulation of insulin secretion",
  "gene_name": "Chromogranin-A",
  "gene_symbol": "CHGA",
  "term_id": "GO:0046676",
  "gene": "UniProtKB:P10645"
}